{
  "gene_symbol": "MYCN",
  "gene_name": "N-myc proto-oncogene protein",
  "term_label": "RNA polymerase II cis-regulatory region sequence-specific DNA binding",
  "gene": "UniProtKB:P04198",
  "term_id": "GO:0000978"
}